{
  "term_label": "nucleus",
  "term_id": "GO:0005634",
  "gene": "UniProtKB:Q9Y4E5",
  "gene_name": "E3 SUMO-protein ligase ZNF451",
  "gene_symbol": "ZNF451"
}